{
  "gene_name": "U3 small nucleolar RNA-associated protein 14 homolog C",
  "term_label": "nucleolus",
  "gene": "UniProtKB:Q5TAP6",
  "term_id": "GO:0005730",
  "gene_symbol": "UTP14C"
}